{
  "gene_name": "Mediator of RNA polymerase II transcription subunit 29",
  "term_id": "GO:0016592",
  "gene": "UniProtKB:Q9NX70",
  "term_label": "mediator complex",
  "gene_symbol": "MED29"
}